negative regulation of metanephric DCT cell differentiation [GO:2000593] (biological process) Sources: GOC:obol Definition: Any process that stops, prevents or reduces the frequency, rate or extent of metanephric DCT cell differentiation. Relationships: is a type of negative regulation of cell differentiation [GO:0045596]; is a type of regulation of metanephric DCT cell differentiation [GO:2000592]; negatively regulates metanephric DCT cell differentiation [GO:0072240] Also known as: negative regulation of metanephric distal convoluted tubule cell differentiation